{
  "term_label": "endosome",
  "term_id": "GO:0005768",
  "gene_symbol": "PI4K2B",
  "gene_name": "Phosphatidylinositol 4-kinase type 2-beta",
  "gene": "UniProtKB:Q8TCG2"
}